beta-lactam antibiotic biosynthetic process [GO:0030654] (biological process) Definition: The chemical reactions and pathways resulting in the formation of a beta-lactam antibiotic, any member of a class of natural or semisynthetic antibiotics whose characteristic feature is a strained, four-membered beta-lactam ring. They include the penicillins and many of the cephalosporins. Sources: GOC:mah, ISBN:0198506732 Also known as: beta-lactam antibiotic anabolism, beta-lactam antibiotic biosynthesis, beta-lactam antibiotic formation, beta-lactam antibiotic synthesis Relationships: is a type of antibiotic biosynthetic process [GO:0017000]; is a type of GO:0072339 Subtypes: penicillin biosynthetic process [GO:0042318], GO:0043646, cephamycin C biosynthetic process [GO:1901118], carbapenem biosynthetic process [GO:1901769]